specification of segmental identity, labial segment [GO:0007381] (BP) Relationships: is a type of GO:0007380; is part of posterior head segmentation [GO:0035289] Definition: The specification of the characteristic structures of the labial segment following establishment of segment boundaries. Identity is considered to be the aggregate of characteristics by which a structure is recognized. Sources: ISBN:0878932437 Note: See also the fly_anatomy.ontology term 'labial segment ; FBbt:00000014'.